{
  "gene_symbol": "CNR1",
  "gene_name": "Cannabinoid receptor 1",
  "term_label": "plasma membrane",
  "gene": "UniProtKB:P21554",
  "term_id": "GO:0005886"
}